negative regulation of natural killer cell degranulation [GO:0043322] (biological process) Also known as: down regulation of natural killer cell degranulation, down-regulation of natural killer cell degranulation, downregulation of natural killer cell degranulation, negative regulation of NK cell degranulation, negative regulation of NK cell granule exocytosis, negative regulation of natural killer cell granule exocytosis, inhibition of natural killer cell degranulation Definition: Any process that stops, prevents, or reduces the rate of natural killer cell degranulation. Sources: ISBN:0781735149 Relationships: is a type of negative regulation of leukocyte degranulation [GO:0043301]; is a type of regulation of natural killer cell degranulation [GO:0043321]; is a type of negative regulation of natural killer cell mediated cytotoxicity [GO:0045953]; negatively regulates natural killer cell degranulation [GO:0043320]